{
  "gene_name": "Katanin p60 ATPase-containing subunit A-like 2",
  "term_label": "cytoplasm",
  "term_id": "GO:0005737",
  "gene_symbol": "KATNAL2",
  "gene": "UniProtKB:Q8IYT4"
}